{
  "gene_name": "Short-chain dehydrogenase_reductase 3",
  "term_label": "regulation of retinoic acid receptor signaling pathway",
  "term_id": "GO:0048385",
  "gene_symbol": "DHRS3",
  "gene": "UniProtKB:O75911"
}